{
  "term_label": "protein folding",
  "term_id": "GO:0006457",
  "gene_symbol": "UNC45B",
  "gene": "UniProtKB:Q8IWX7",
  "gene_name": "Protein unc-45 homolog B"
}